{
  "term_id": "GO:0006805",
  "term_label": "xenobiotic metabolic process",
  "gene_symbol": "CYP2W1",
  "gene": "UniProtKB:Q8TAV3",
  "gene_name": "Cytochrome P450 2W1"
}